{
  "gene": "UniProtKB:O60674",
  "gene_symbol": "JAK2",
  "term_label": "non-membrane spanning protein tyrosine kinase activity",
  "gene_name": "Tyrosine-protein kinase JAK2",
  "term_id": "GO:0004715"
}